{
  "gene_symbol": "ANKRD45",
  "gene": "UniProtKB:Q5TZF3",
  "term_label": "Unknown molecular function",
  "gene_name": "Ankyrin repeat domain-containing protein 45",
  "term_id": "UNKNOWN:0001"
}